{
  "gene_symbol": "THY1",
  "gene_name": "Thy-1 membrane glycoprotein",
  "term_label": "integrin-mediated signaling pathway",
  "gene": "UniProtKB:P04216",
  "term_id": "GO:0007229"
}